{
  "gene": "UniProtKB:Q7L8J4",
  "term_label": "protein kinase inhibitor activity",
  "term_id": "GO:0004860",
  "gene_symbol": "SH3BP5L",
  "gene_name": "SH3 domain-binding protein 5-like"
}